{
  "gene": "UniProtKB:P35558",
  "term_id": "GO:0032869",
  "gene_name": "Phosphoenolpyruvate carboxykinase, cytosolic [GTP]",
  "gene_symbol": "PCK1",
  "term_label": "cellular response to insulin stimulus"
}